{
  "term_id": "GO:0007186",
  "gene": "UniProtKB:P35410",
  "gene_name": "Mas-related G-protein coupled receptor MRG",
  "gene_symbol": "MAS1L",
  "term_label": "G protein-coupled receptor signaling pathway"
}